omega-hydroxydecanoate dehydrogenase activity [GO:0050153] (molecular function) Relationships: is a type of GO:0016616 Sources: EC:1.1.1.66, RHEA:20880 Also known as: w-hydroxydecanoate dehydrogenase activity, 10-hydroxydecanoate:NAD+ 10-oxidoreductase activity Definition: Catalysis of the reaction: 10-hydroxydecanoate + NAD+ = 10-oxodecanoate + H+ + NADH.